{
  "term_id": "GO:0005178",
  "gene": "UniProtKB:O76076",
  "gene_name": "CCN family member 5",
  "term_label": "integrin binding",
  "gene_symbol": "CCN5"
}